{
  "gene": "UniProtKB:P16619",
  "gene_symbol": "CCL3L1",
  "gene_name": "C-C motif chemokine 3-like 1",
  "term_id": "GO:0070098",
  "term_label": "chemokine-mediated signaling pathway"
}